{
  "gene_symbol": "KRTAP5-3",
  "gene_name": "Keratin-associated protein 5-3",
  "term_id": "UNKNOWN:0003",
  "term_label": "Unknown cellular component",
  "gene": "UniProtKB:Q6L8H2"
}